{
  "gene_name": "Ribosome biogenesis protein NOP53",
  "term_id": "GO:0005730",
  "term_label": "nucleolus",
  "gene": "UniProtKB:Q9NZM5",
  "gene_symbol": "NOP53"
}